rod telodendria [GO:0120210] (cellular component) Relationships: is a type of telodendria [GO:0120208] References: PMID:14755521 Sources: GOC:cvs, GOC:krc Definition: Rod telodendria are projections that originate from the rod pedicle and form gap junctions with other photoreceptors within the outer plexiform layer of the retina.